{
  "term_label": "ERAD pathway",
  "gene_symbol": "UFD1",
  "gene_name": "Ubiquitin recognition factor in ER-associated degradation protein 1",
  "term_id": "GO:0036503",
  "gene": "UniProtKB:Q92890"
}